{
  "gene_name": "Transcription factor COE2",
  "gene": "UniProtKB:Q9HAK2",
  "term_id": "GO:0000981",
  "term_label": "DNA-binding transcription factor activity, RNA polymerase II-specific",
  "gene_symbol": "EBF2"
}